{
  "term_label": "Unknown molecular function",
  "gene": "UniProtKB:Q9BZA5",
  "term_id": "UNKNOWN:0001",
  "gene_name": "Putative gamma-taxilin 2",
  "gene_symbol": "TXLNGY"
}